{
  "gene_symbol": "RBMX",
  "gene": "UniProtKB:P38159",
  "gene_name": "RNA-binding motif protein, X chromosome",
  "term_id": "GO:0003729",
  "term_label": "mRNA binding"
}